{
  "gene": "UniProtKB:Q99575",
  "gene_name": "Ribonucleases P_MRP protein subunit POP1",
  "gene_symbol": "POP1",
  "term_label": "ribonuclease MRP complex",
  "term_id": "GO:0000172"
}